ribosomal large subunit biogenesis [GO:0042273] (biological process) Sources: GOC:jl Relationships: is a type of ribonucleoprotein complex biogenesis [GO:0022613]; is part of ribosome biogenesis [GO:0042254] Definition: A cellular process that results in the biosynthesis of constituent macromolecules, assembly, and arrangement of constituent parts of a large ribosomal subunit; includes transport to the sites of protein synthesis. Also known as: ribosomal large subunit biogenesis and assembly